{
  "term_label": "bicellular tight junction",
  "gene_name": "Putative claudin-25",
  "gene": "UniProtKB:C9JDP6",
  "gene_symbol": "CLDN25",
  "term_id": "GO:0005923"
}